{
  "gene_symbol": "MMP8",
  "term_label": "extracellular matrix organization",
  "gene_name": "Neutrophil collagenase",
  "term_id": "GO:0030198",
  "gene": "UniProtKB:P22894"
}